{
  "gene_symbol": "PPHLN1",
  "gene": "UniProtKB:Q8NEY8",
  "term_id": "UNKNOWN:0001",
  "term_label": "Unknown molecular function",
  "gene_name": "Periphilin-1"
}